myrcene synthase activity [GO:0050551] (molecular function) Sources: EC:4.2.3.15, RHEA:16965 Definition: Catalysis of the reaction: geranyl diphosphate = diphosphate + myrcene. Relationships: is a type of terpene synthase activity [GO:0010333] Also known as: geranyl-diphosphate diphosphate-lyase (myrcene-forming) activity